{
  "gene": "UniProtKB:Q9Y3E7",
  "term_id": "GO:0032509",
  "gene_symbol": "CHMP3",
  "gene_name": "Charged multivesicular body protein 3",
  "term_label": "endosome transport via multivesicular body sorting pathway"
}